negative regulation of chlorophyll catabolic process [GO:1903647] (biological process) Definition: Any process that stops, prevents or reduces the frequency, rate or extent of chlorophyll catabolic process. Relationships: is a type of regulation of chlorophyll catabolic process [GO:0010271]; is a type of GO:1901405; negatively regulates chlorophyll catabolic process [GO:0015996] Also known as: down regulation of chlorophyll breakdown, down regulation of chlorophyll catabolic process, down regulation of chlorophyll catabolism, down regulation of chlorophyll degradation, down-regulation of chlorophyll breakdown, down-regulation of chlorophyll catabolic process, down-regulation of chlorophyll catabolism, down-regulation of chlorophyll degradation, downregulation of chlorophyll breakdown, downregulation of chlorophyll catabolic process, downregulation of chlorophyll catabolism, downregulation of chlorophyll degradation, negative regulation of chlorophyll breakdown, negative regulation of chlorophyll catabolism, negative regulation of chlorophyll degradation, inhibition of chlorophyll breakdown, inhibition of chlorophyll catabolic process, inhibition of chlorophyll catabolism, inhibition of chlorophyll degradation References: PMID:24719469 Sources: GOC:TermGenie, GO_REF:0000058